positive regulation of sclerotome development [GO:0061189] (biological process) Relationships: is a type of positive regulation of developmental process [GO:0051094]; is a type of regulation of sclerotome development [GO:0061190]; positively regulates sclerotome development [GO:0061056] Definition: Any process that increases the rate, frequency, or extent of the progression of the sclerotome over time, from its initial formation to the mature structure. The sclerotome is the portion of the somite that will give rise to a vertebra. Sources: GOC:BHF, GOC:dph